{
  "gene": "UniProtKB:P25054",
  "term_label": "pattern specification process",
  "term_id": "GO:0007389",
  "gene_symbol": "APC",
  "gene_name": "Adenomatous polyposis coli protein"
}